{
  "gene": "UniProtKB:Q8WW33",
  "term_label": "Unknown cellular component",
  "term_id": "UNKNOWN:0003",
  "gene_symbol": "GTSF1",
  "gene_name": "Gametocyte-specific factor 1"
}